{
  "gene": "UniProtKB:Q58FF8",
  "term_id": "GO:0048471",
  "gene_name": "Putative heat shock protein HSP 90-beta 2",
  "term_label": "perinuclear region of cytoplasm",
  "gene_symbol": "HSP90AB2P"
}